{
  "gene": "UniProtKB:P55957",
  "term_label": "positive regulation of extrinsic apoptotic signaling pathway",
  "term_id": "GO:2001238",
  "gene_name": "BH3-interacting domain death agonist",
  "gene_symbol": "BID"
}